{
  "gene": "UniProtKB:Q9BVL2",
  "term_id": "GO:0005643",
  "term_label": "nuclear pore",
  "gene_symbol": "NUP58",
  "gene_name": "Nucleoporin p58_p45"
}